{
  "term_label": "Unknown biological process",
  "term_id": "UNKNOWN:0002",
  "gene_symbol": "METAP1",
  "gene": "UniProtKB:P53582",
  "gene_name": "Methionine aminopeptidase 1"
}